actin polymerization-dependent cell motility [GO:0070358] (biological process) Definition: A process involved in the controlled movement of a bacterial cell powered by the continuous polymerization of actin at one pole of the cell. Also known as: cell motility by actin tail formation Subtypes: symbiont-mediated actin polymerization-dependent cell-to-cell migration in host [GO:0070360] References: PMID:15773977 Sources: GOC:mah Relationships: is a type of GO:0048870